rRNA primary transcript binding [GO:0042134] (molecular function) Also known as: pre-rRNA binding Sources: GOC:jl Definition: Binding to an unprocessed ribosomal RNA transcript. Relationships: is a type of rRNA binding [GO:0019843]